{
  "term_id": "GO:0009898",
  "gene_name": "Charged multivesicular body protein 7",
  "gene_symbol": "CHMP7",
  "gene": "UniProtKB:Q8WUX9",
  "term_label": "cytoplasmic side of plasma membrane"
}